base-excision repair, AP site formation [GO:0006285] (biological process) Sources: ISBN:0815316194 Subtypes: depurination [GO:0045007], depyrimidination [GO:0045008], base-excision repair, AP site formation via deaminated base removal [GO:0097510] Definition: The formation of an AP site, a deoxyribose sugar with a missing base, by DNA glycosylase which recognizes an altered base in DNA and catalyzes its hydrolytic removal. This sugar phosphate is the substrate recognized by the AP endonuclease, which cuts the DNA phosphodiester backbone at the 5' side of the altered site to leave a gap which is subsequently repaired. Relationships: is a type of GO:0006259; BFO_0000050 base-excision repair [GO:0006284]